regulation of gliogenesis [GO:0014013] (BP) Definition: Any process that modulates the frequency, rate or extent of gliogenesis, the formation of mature glia. Sources: GOC:ef Relationships: is_a GO:0050767; regulates GO:0042063 Subtypes: negative regulation of gliogenesis [GO:0014014], positive regulation of gliogenesis [GO:0014015]